protein-DNA-RNA complex remodeling [GO:0001119] (biological process) Sources: GOC:txnOH Definition: The acquisition, loss, or modification of macromolecules within a protein-DNA-RNA complex, resulting in the alteration of an existing complex. Relationships: is a type of GO:0001115; is a type of protein-containing complex remodeling [GO:0034367]